{
  "term_label": "protein-RNA sequence-specific adaptor activity",
  "gene_name": "mRNA decay activator protein ZFP36L2",
  "term_id": "GO:0160134",
  "gene": "UniProtKB:P47974",
  "gene_symbol": "ZFP36L2"
}